positive regulation of telomere maintenance [GO:0032206] (biological process) Definition: Any process that activates or increases the frequency, rate or extent of a process that affects and monitors the activity of telomeric proteins and the length of telomeric DNA. Subtypes: positive regulation of telomere maintenance via recombination [GO:0032209], positive regulation of telomere maintenance via semi-conservative replication [GO:0032215], positive regulation of telomere capping [GO:1904355], positive regulation of telomere maintenance via telomere lengthening [GO:1904358], positive regulation of telomeric loop formation [GO:1904420], positive regulation of t-circle formation [GO:1904431], GO:1904507, positive regulation of telomeric loop disassembly [GO:1904535] Relationships: is a type of regulation of telomere maintenance [GO:0032204]; is a type of GO:0051054; is a type of positive regulation of chromosome organization [GO:2001252]; positively regulates telomere maintenance [GO:0000723] Sources: GOC:mah Also known as: up regulation of telomere maintenance, up-regulation of telomere maintenance, upregulation of telomere maintenance, activation of telomere maintenance, stimulation of telomere maintenance